{
  "gene": "UniProtKB:Q9NRJ1",
  "gene_symbol": "C8orf17",
  "term_id": "UNKNOWN:0002",
  "gene_name": "Protein MOST-1",
  "term_label": "Unknown biological process"
}